deoxyribose phosphate biosynthetic process [GO:0046385] (biological process) Relationships: is a type of phosphate-containing compound metabolic process [GO:0006796]; is a type of organophosphate biosynthetic process [GO:0090407]; is a type of GO:1901137 Also known as: deoxyribose phosphate anabolism, deoxyribose phosphate biosynthesis, deoxyribose phosphate formation, deoxyribose phosphate synthesis Subtypes: 2-deoxyribose 1-phosphate biosynthetic process [GO:0006016], 2'-deoxyribonucleotide biosynthetic process [GO:0009265] Sources: ISBN:0198506732 Definition: The chemical reactions and pathways resulting in the formation of deoxyribose phosphate, the phosphorylated sugar 2-deoxy-erythro-pentose.